kisspeptin receptor binding [GO:0031773] (molecular function) Sources: GOC:mah, GOC:nln Also known as: G-protein coupled receptor 54 binding, KiSS-1 receptor binding, hOT7T175 receptor binding, hypogonadotropin-1 receptor binding, metastin receptor binding, kisspeptin receptor ligand Definition: Binding to a kisspeptin receptor. Relationships: is a type of neuropeptide receptor binding [GO:0071855]